{
  "gene_symbol": "TRIQK",
  "term_id": "UNKNOWN:0002",
  "gene": "UniProtKB:Q629K1",
  "term_label": "Unknown biological process",
  "gene_name": "Triple QxxK_R motif-containing protein"
}